{
  "gene_symbol": "POLE2",
  "gene_name": "DNA polymerase epsilon subunit 2",
  "gene": "UniProtKB:P56282",
  "term_id": "GO:0008622",
  "term_label": "epsilon DNA polymerase complex"
}